{
  "gene_name": "WD repeat domain-containing protein 83",
  "gene": "UniProtKB:Q9BRX9",
  "term_id": "GO:0071013",
  "term_label": "catalytic step 2 spliceosome",
  "gene_symbol": "WDR83"
}